{
  "gene_name": "AF4_FMR2 family member 3",
  "gene": "UniProtKB:P51826",
  "gene_symbol": "AFF3",
  "term_label": "transcription coregulator activity",
  "term_id": "GO:0003712"
}